voltage-gated calcium channel activity involved SA node cell action potential [GO:0086059] (molecular function) Definition: Enables the transmembrane transfer of a calcium ion by a voltage-gated channel across the plasma membrane of an SA node cardiac muscle cell that contributes to the depolarization phase of an action potential. A voltage-gated channel is a channel whose open state is dependent on the voltage across the membrane in which it is embedded. Relationships: is a type of voltage-gated calcium channel activity involved in cardiac muscle cell action potential [GO:0086007]; is part of membrane depolarization during SA node cell action potential [GO:0086046] Sources: GOC:BHF, GOC:mtg_cardiac_conduct_nov11 Also known as: voltage-gated calcium channel activity involved in SA node cardiac muscle cell action potential, voltage-gated calcium channel activity involved in SAN cardiac muscle cell action potential, voltage-gated calcium channel activity involved in sinoatrial node cardiac muscle cell action potential, voltage-gated calcium channel activity involved in sinus node cardiac muscle cell action potential